diakinesis [GO:0000241] (biological process) Sources: GOC:mtg_cell_cycle Relationships: is a type of meiosis I cell cycle phase [GO:0098764]; is part of meiotic prophase I [GO:0007128] Note: Note that this term should not be used for direct annotation. If you are trying to make an annotation to x phase, it is likely that the correct annotation is 'regulation of x/y phase transition' or to a process which occurs during the reported phase (i.e mitotic DNA replication for mitotic S-phase). To capture the phase when a specific location or process is observed, the phase term can be used in an annotation extension (PMID:24885854) applied to a cellular component term (with the relation exists_during) or a biological process term (with the relation happens_during). Definition: The cell cycle phase which follows diplotene during prophase I of meiosis, the separation of homologous chromosomes is complete and crossing over has occurred.